{
  "term_id": "GO:0005347",
  "gene_symbol": "SLC25A24",
  "term_label": "ATP transmembrane transporter activity",
  "gene": "UniProtKB:Q6NUK1",
  "gene_name": "Mitochondrial adenyl nucleotide antiporter SLC25A24"
}